{
  "gene_name": "Putative uncharacterized protein C5orf58",
  "gene": "UniProtKB:C9J3I9",
  "gene_symbol": "C5orf58",
  "term_id": "UNKNOWN:0003",
  "term_label": "Unknown cellular component"
}